type 1 cannabinoid receptor binding [GO:0031718] (molecular function) Sources: GOC:mah, GOC:nln Relationships: is a type of cannabinoid receptor binding [GO:0031717] Definition: Binding to a type 1 cannabinoid receptor. Also known as: type 1 cannabinoid receptor ligand